{
  "term_id": "GO:0015811",
  "gene": "UniProtKB:P82251",
  "term_label": "L-cystine transport",
  "gene_symbol": "SLC7A9",
  "gene_name": "b(0,+)-type amino acid transporter 1"
}